{
  "gene_name": "Transcription factor SOX-10",
  "term_id": "GO:0048484",
  "term_label": "enteric nervous system development",
  "gene": "UniProtKB:P56693",
  "gene_symbol": "SOX10"
}